{
  "gene_name": "Sperm-associated antigen 8",
  "term_id": "GO:0045944",
  "gene": "UniProtKB:Q99932",
  "term_label": "positive regulation of transcription by RNA polymerase II",
  "gene_symbol": "SPAG8"
}